positive regulation of defense response to insect [GO:1900367] (biological process) Relationships: is a type of positive regulation of response to biotic stimulus [GO:0002833]; is a type of positive regulation of defense response [GO:0031349]; is a type of positive regulation of response to external stimulus [GO:0032103]; is a type of regulation of defense response to insect [GO:2000068]; positively regulates defense response to insect [GO:0002213] Definition: Any process that activates or increases the frequency, rate or extent of defense response to insect. Also known as: positive regulation of physiological defense response to insect, up regulation of defense response to insect, up regulation of physiological defense response to insect, up-regulation of defense response to insect, up-regulation of physiological defense response to insect, upregulation of defense response to insect, upregulation of physiological defense response to insect, activation of defense response to insect, activation of physiological defense response to insect References: PMID:22474183 Sources: GOC:TermGenie